{
  "term_label": "histone binding",
  "gene_name": "Testis-specific Y-encoded protein 3",
  "term_id": "GO:0042393",
  "gene_symbol": "TSPY3",
  "gene": "UniProtKB:P0CV98"
}